bursicon neuropeptide hormone complex [GO:0031395] (cellular component) Relationships: is a type of protein-containing complex [GO:0032991]; is part of GO:0005576 Sources: GOC:rc Definition: A neuropeptide hormone secreted by the central nervous system of insects that stimulates the tanning and sclerotization of the adult cuticle following eclosion. The active hormone consists of an obligate heterodimer of the alpha and beta subunits.